{
  "term_id": "GO:0003836",
  "gene_symbol": "ST3GAL4",
  "gene_name": "CMP-N-acetylneuraminate-beta-galactosamide-alpha-2,3-sialyltransferase 4",
  "gene": "UniProtKB:Q11206",
  "term_label": "beta-galactoside (CMP) alpha-2,3-sialyltransferase activity"
}